{
  "gene_symbol": "LRP10",
  "term_id": "GO:0005041",
  "gene_name": "Low-density lipoprotein receptor-related protein 10",
  "gene": "UniProtKB:Q7Z4F1",
  "term_label": "low-density lipoprotein particle receptor activity"
}